high-affinity L-ornithine transmembrane transporter activity [GO:0097627] (molecular function) Also known as: high affinity L-ornithine transmembrane transporter activity Definition: Enables the transfer of L-ornithine from one side of a membrane to the other. In high-affinity transport the transporter is able to bind the solute even if it is only present at very low concentrations. References: PMID:8195186 Sources: GOC:krc Relationships: is a type of L-ornithine transmembrane transporter activity [GO:0000064]